histone H3R17 arginine deiminase activity [GO:0140797] (molecular function) Relationships: is a type of GO:0141057 Definition: Catalysis of the reaction: H2O + histone H3 L-arginyl (position 17)= histone H3 L-citrullyl (position 17) + NH4+, resulting in histone H3 citrullination at position 17. Note: Comment: Note that the residue position corresponds to the canonical human H3 histone (UniProtKB:P84243); this residue is conserved across all eukaryotes. Residue 1 is the first residue following removal of the initiating Methionine (Met). Note that each histone is encoded by multiple genes, and sequences may vary across different genes within an organism. The substrate for histone deiminase may be methyl-arginine, rather than arginine (see PMID:35197210 and PMID:16567635). References: PMID:15339660 Also known as: H3-R17 citrullination, histone H3-R17 arginine deiminase activity, histone-arginine deiminase activity (H3-R17 specific)